{
  "gene": "UniProtKB:P51398",
  "term_label": "Unknown biological process",
  "term_id": "UNKNOWN:0002",
  "gene_name": "Small ribosomal subunit protein mS29",
  "gene_symbol": "DAP3"
}